{
  "gene_symbol": "MARK2",
  "gene_name": "Serine_threonine-protein kinase MARK2",
  "gene": "UniProtKB:Q7KZI7",
  "term_id": "GO:0035556",
  "term_label": "intracellular signal transduction"
}